{
  "gene_symbol": "GSAP",
  "gene_name": "Gamma-secretase-activating protein",
  "term_id": "GO:0005802",
  "term_label": "trans-Golgi network",
  "gene": "UniProtKB:A4D1B5"
}